DNA polymerase V complex [GO:0009355] (cellular component) References: PMID:10430871, PMID:10542196 Relationships: is a type of DNA polymerase complex [GO:0042575] Definition: A DNA polymerase complex that contains two UmuD' and one UmuC subunits, and acts in translesion DNA synthesis.